{
  "gene": "UniProtKB:Q6NT52",
  "gene_name": "Choriogonadotropin subunit beta variant 2",
  "gene_symbol": "CGB2",
  "term_label": "G protein-coupled receptor signaling pathway",
  "term_id": "GO:0007186"
}